{
  "gene": "UniProtKB:Q9BPY8",
  "term_label": "nucleus",
  "gene_symbol": "HOPX",
  "term_id": "GO:0005634",
  "gene_name": "Homeodomain-only protein"
}